{
  "gene_symbol": "CCL15",
  "gene": "UniProtKB:Q16663",
  "gene_name": "C-C motif chemokine 15",
  "term_id": "GO:0008009",
  "term_label": "chemokine activity"
}